{
  "gene_symbol": "DDAH2",
  "gene": "UniProtKB:O95865",
  "term_label": "mitochondrion",
  "term_id": "GO:0005739",
  "gene_name": "N(G),N(G)-dimethylarginine dimethylaminohydrolase 2"
}